{
  "gene": "UniProtKB:Q1W209",
  "gene_symbol": "ESRG",
  "gene_name": "Embryonic stem cell-related gene protein",
  "term_id": "UNKNOWN:0002",
  "term_label": "Unknown biological process"
}